{
  "gene_symbol": "AOC1",
  "term_id": "GO:0008131",
  "gene": "UniProtKB:P19801",
  "gene_name": "Amiloride-sensitive amine oxidase [copper-containing]",
  "term_label": "primary methylamine oxidase activity"
}